{
  "gene_symbol": "MTCL1",
  "term_id": "GO:0097427",
  "gene": "UniProtKB:Q9Y4B5",
  "term_label": "microtubule bundle",
  "gene_name": "Microtubule cross-linking factor 1"
}